{
  "term_label": "epidermal growth factor receptor signaling pathway",
  "gene_name": "Probetacellulin",
  "gene_symbol": "BTC",
  "term_id": "GO:0007173",
  "gene": "UniProtKB:P35070"
}